regulation of pronephric nephron tubule development [GO:1900206] (biological process) Sources: GOC:TermGenie Relationships: is a type of regulation of developmental process [GO:0050793]; regulates pronephric nephron tubule development [GO:0039020] Definition: Any process that modulates the frequency, rate or extent of pronephric nephron tubule development. Subtypes: negative regulation of pronephric nephron tubule development [GO:1900207]